{
  "term_id": "GO:0008236",
  "term_label": "serine-type peptidase activity",
  "gene": "UniProtKB:P98073",
  "gene_name": "Enteropeptidase",
  "gene_symbol": "TMPRSS15"
}